{
  "term_label": "integrin-mediated signaling pathway",
  "term_id": "GO:0007229",
  "gene": "UniProtKB:P08514",
  "gene_name": "Integrin alpha-IIb",
  "gene_symbol": "ITGA2B"
}